{
  "term_label": "extracellular region",
  "gene_symbol": "ANGPTL8",
  "term_id": "GO:0005576",
  "gene_name": "Angiopoietin-like protein 8",
  "gene": "UniProtKB:Q6UXH0"
}